{
  "term_id": "UNKNOWN:0003",
  "gene": "UniProtKB:Q8N7L0",
  "term_label": "Unknown cellular component",
  "gene_symbol": "FAM216B",
  "gene_name": "Protein FAM216B"
}